very-low-density lipoprotein particle remodeling [GO:0034372] (biological process) Sources: GOC:BHF, GOC:expert_pt, GOC:mah, GOC:rl Regulation: regulated by GO:0010901; RO_0002213 by positive regulation of very-low-density lipoprotein particle remodeling [GO:0010902]; negatively regulated by negative regulation of very-low-density lipoprotein particle remodeling [GO:0010903] Definition: The acquisition, loss or modification of a protein or lipid within a very-low-density lipoprotein particle, including the hydrolysis of triglyceride by hepatic lipase or lipoprotein lipase and the subsequent loss of free fatty acid. Relationships: is a type of triglyceride-rich lipoprotein particle remodeling [GO:0034370] Also known as: VDL remodeling, VDL remodelling, very-low-density lipoprotein particle remodelling, VDL formation